{
  "term_label": "P-type sodium:potassium-exchanging transporter activity",
  "term_id": "GO:0005391",
  "gene": "UniProtKB:P54707",
  "gene_symbol": "ATP12A",
  "gene_name": "Potassium-transporting ATPase alpha chain 2"
}